U2 snRNP [GO:0005686] (cellular component) Also known as: snRNP U2, 17S U2 snRNP Sources: GOC:krc, GOC:mah, ISBN:0879695897 Note: U2 snRNP refers to the U2 small nuclear RNA and the proteins that associate with it. U2 snRNP is not considered to be a type of spliceosomal complex by itself. Definition: A ribonucleoprotein complex that contains small nuclear RNA U2, a heptameric ring of Sm proteins, as well as several proteins that are unique to the U2 snRNP, most of which remain associated with the U2 snRNA both while the U2 snRNP is free or assembled into a series of spliceosomal complexes. Relationships: is a type of spliceosomal snRNP complex [GO:0097525]